{
  "term_label": "leukocyte tethering or rolling",
  "gene": "UniProtKB:Q9NZ53",
  "gene_name": "Podocalyxin-like protein 2",
  "gene_symbol": "PODXL2",
  "term_id": "GO:0050901"
}